{
  "term_id": "GO:0005886",
  "gene_name": "Type-2 angiotensin II receptor",
  "gene": "UniProtKB:P50052",
  "term_label": "plasma membrane",
  "gene_symbol": "AGTR2"
}